{
  "gene": "UniProtKB:P54368",
  "gene_name": "Ornithine decarboxylase antizyme 1",
  "term_id": "GO:0005634",
  "term_label": "nucleus",
  "gene_symbol": "OAZ1"
}